{
  "gene_symbol": "COLQ",
  "term_label": "heparin binding",
  "gene": "UniProtKB:Q9Y215",
  "gene_name": "Acetylcholinesterase collagenic tail peptide",
  "term_id": "GO:0008201"
}